{
  "gene_name": "SH2B adapter protein 3",
  "term_id": "GO:0060761",
  "gene": "UniProtKB:Q9UQQ2",
  "gene_symbol": "SH2B3",
  "term_label": "negative regulation of response to cytokine stimulus"
}